{
  "gene_symbol": "KCNH7",
  "gene_name": "Potassium voltage-gated channel subfamily H member 7",
  "gene": "UniProtKB:Q9NS40",
  "term_id": "GO:0005242",
  "term_label": "inward rectifier potassium channel activity"
}